arabinogalactan endo-1,4-beta-galactosidase activity [GO:0031218] (molecular function) Definition: Catalysis of the endohydrolysis of (1->4)-beta-D-galactosidic linkages in arabinogalactans. Sources: EC:3.2.1.89, GOC:mlg Also known as: arabinogalactanase activity, endo-1,4-beta-galactanase activity, galactanase activity, arabinogalactan 4-beta-D-galactanohydrolase activity Relationships: is_a galactosidase activity [GO:0015925]